transport vesicle lumen [GO:0098566] (cellular component) Sources: GOC:dos Definition: The volume enclosed within the membrane of a transport vesicle. Subtypes: GO:0062246, trans-Golgi network transport vesicle lumen [GO:0098564] Relationships: is a type of cytoplasmic vesicle lumen [GO:0060205]; is part of transport vesicle [GO:0030133]